muscle tissue development [GO:0060537] (BP) Regulation: regulated by regulation of muscle tissue development [GO:1901861]; negatively regulated by negative regulation of muscle tissue development [GO:1901862]; positively regulated by GO:1901863 Relationships: is a type of tissue development [GO:0009888] Subtypes: striated muscle tissue development [GO:0014706], smooth muscle tissue development [GO:0048745] Sources: GOC:dph Definition: The progression of muscle tissue over time, from its initial formation to its mature state. Muscle tissue is a contractile tissue made up of actin and myosin fibers.